{
  "gene_name": "Putative uncharacterized protein MYH16",
  "term_label": "Unknown biological process",
  "gene": "UniProtKB:Q9H6N6",
  "term_id": "UNKNOWN:0002",
  "gene_symbol": "MYH16"
}